{
  "gene": "UniProtKB:Q8TDF6",
  "term_label": "plasma membrane",
  "gene_name": "RAS guanyl-releasing protein 4",
  "gene_symbol": "RASGRP4",
  "term_id": "GO:0005886"
}